{
  "term_label": "Toll signaling pathway",
  "gene_symbol": "MYD88",
  "term_id": "GO:0008063",
  "gene_name": "Myeloid differentiation primary response protein MyD88",
  "gene": "UniProtKB:Q99836"
}